efferent axon development in anterior lateral line nerve [GO:0048911] (biological process) Relationships: is a type of efferent axon development in a lateral line nerve [GO:0048894]; is part of GO:0048909 Definition: The process whose specific outcome is the progression of an efferent axon in the anterior lateral line nerve over time from its formation to the mature structure. This process includes axonogenesis and pathfinding of the efferent axons in the anterior lateral line nerve. References: PMID:15018940